{
  "gene_symbol": "RBM45",
  "term_label": "ribonucleoprotein complex",
  "gene": "UniProtKB:Q8IUH3",
  "gene_name": "RNA-binding protein 45",
  "term_id": "GO:1990904"
}